{
  "gene_symbol": "NPM1",
  "gene": "UniProtKB:P06748",
  "gene_name": "Nucleophosmin",
  "term_id": "GO:0042393",
  "term_label": "histone binding"
}